regulation of stomatal complex patterning [GO:2000037] (biological process) Definition: Any process that modulates the frequency, rate or extent of stomatal complex patterning. Sources: GOC:obol Relationships: is a type of regulation of multicellular organismal process [GO:0051239]; regulates stomatal complex patterning [GO:0010375]